{
  "term_label": "sex differentiation",
  "gene_name": "Doublesex- and mab-3-related transcription factor 2",
  "gene_symbol": "DMRT2",
  "term_id": "GO:0007548",
  "gene": "UniProtKB:Q9Y5R5"
}